{
  "gene_symbol": "MEIS2",
  "term_label": "RNA polymerase II cis-regulatory region sequence-specific DNA binding",
  "gene": "UniProtKB:O14770",
  "gene_name": "Homeobox protein Meis2",
  "term_id": "GO:0000978"
}